{
  "gene": "UniProtKB:O75973",
  "term_label": "Unknown molecular function",
  "gene_symbol": "C1QL1",
  "gene_name": "C1q-related factor",
  "term_id": "UNKNOWN:0001"
}